{
  "term_id": "GO:0031639",
  "gene_name": "Tissue-type plasminogen activator",
  "gene_symbol": "PLAT",
  "gene": "UniProtKB:P00750",
  "term_label": "plasminogen activation"
}